{
  "gene_symbol": "POU4F3",
  "term_id": "GO:0000978",
  "gene_name": "POU domain, class 4, transcription factor 3",
  "gene": "UniProtKB:Q15319",
  "term_label": "RNA polymerase II cis-regulatory region sequence-specific DNA binding"
}